positive regulation of synaptic vesicle clustering [GO:2000809] (biological process) Relationships: is a type of positive regulation of transport [GO:0051050]; is a type of GO:2000807; positively regulates synaptic vesicle clustering [GO:0097091] Definition: Any process that activates or increases the frequency, rate or extent of synaptic vesicle clustering. References: PMID:21513708